{
  "gene_name": "YjeF N-terminal domain-containing protein 3",
  "gene_symbol": "YJEFN3",
  "term_id": "GO:0005739",
  "term_label": "mitochondrion",
  "gene": "UniProtKB:A6XGL0"
}